{
  "gene_symbol": "NUAK2",
  "term_label": "Unknown cellular component",
  "term_id": "UNKNOWN:0003",
  "gene_name": "NUAK family SNF1-like kinase 2",
  "gene": "UniProtKB:Q9H093"
}